unicellular trichome tip [GO:0090553] (cellular component) Sources: GOC:PO_curators Relationships: is a type of GO:0110165; BFO_0000050 unicellular trichome apex [GO:0090552] Definition: A cell projection part that is the apical most portion of a unicellular trichome apex.